peroxisome membrane targeting sequence binding [GO:0033328] (molecular function) Relationships: is a type of peroxisome targeting sequence binding [GO:0000268] Subtypes: peroxisome membrane class-1 targeting sequence binding [GO:0036105], peroxisome membrane class-2 targeting sequence binding [GO:0036106] Definition: Binding to a peroxisomal membrane targeting sequence, any of several sequences of amino acids within a protein that can act as a signal for the localization of the protein into the peroxisome membrane. Also known as: PMP targeting signal (mPTS) binding, PMP targeting signal binding, mPTS binding, peroxisomal membrane protein (PMP) targeting signal (mPTS) binding References: PMID:15133130, PMID:17020786 Sources: GOC:rb